pyrimidine deoxyribonucleotide binding [GO:0032556] (molecular function) Relationships: is_a GO:0019103; is a type of deoxyribonucleotide binding [GO:0032552] Sources: GOC:mah Definition: Binding to a pyrimidine deoxyribonucleotide, any compound consisting of a pyrimidine deoxyribonucleoside that is esterified with (ortho)phosphate or an oligophosphate at any hydroxyl group on the deoxyribose moiety.